{
  "term_id": "GO:0004144",
  "gene": "UniProtKB:Q3SYC2",
  "gene_name": "2-acylglycerol O-acyltransferase 2",
  "gene_symbol": "MOGAT2",
  "term_label": "diacylglycerol O-acyltransferase activity"
}